{
  "gene_name": "F-box only protein 16",
  "gene": "UniProtKB:Q8IX29",
  "term_id": "UNKNOWN:0002",
  "gene_symbol": "FBXO16",
  "term_label": "Unknown biological process"
}